short-term memory [GO:0007614] (biological process) Relationships: is a type of memory [GO:0007613] Sources: ISBN:0582227089, http://hebb.mit.edu/courses/9.03/lecture4.html Definition: The memory process that deals with the storage, retrieval and modification of information received a short time (up to about 30 minutes) ago. This type of memory is typically dependent on direct, transient effects of second messenger activation.